{
  "term_label": "hippo signaling",
  "term_id": "GO:0035329",
  "gene_symbol": "LATS2",
  "gene": "UniProtKB:Q9NRM7",
  "gene_name": "Serine_threonine-protein kinase LATS2"
}